{
  "term_label": "cytoskeleton organization",
  "gene_symbol": "SORBS1",
  "gene": "UniProtKB:Q9BX66",
  "gene_name": "Sorbin and SH3 domain-containing protein 1",
  "term_id": "GO:0007010"
}